{
  "gene_name": "T cell receptor alpha joining 32 (Fragment)",
  "gene_symbol": "TRAJ32",
  "term_label": "Unknown biological process",
  "gene": "UniProtKB:A0A075B6X3",
  "term_id": "UNKNOWN:0002"
}